regulation of coagulation [GO:0050818] (biological process) Sources: GOC:ai Definition: Any process that modulates the frequency, rate or extent of coagulation, the process in which a fluid solution, or part of it, changes into a solid or semisolid mass. Also known as: regulation of clotting Relationships: is a type of regulation of multicellular organismal process [GO:0051239]; regulates coagulation [GO:0050817] Subtypes: regulation of blood coagulation [GO:0030193], negative regulation of coagulation [GO:0050819], positive regulation of coagulation [GO:0050820]